{
  "term_id": "UNKNOWN:0003",
  "gene": "UniProtKB:Q9NXS2",
  "gene_symbol": "QPCTL",
  "term_label": "Unknown cellular component",
  "gene_name": "Glutaminyl-peptide cyclotransferase-like protein"
}